GDP-mannose hydrolase activity [GO:0052751] (molecular function) Definition: Catalysis of the reaction: GDP-mannose + H2O = GMP + mannose-1-phosphate. Also known as: GDP-mannose pyrophosphatase activity References: PMID:16766526 Relationships: is a type of GO:0016462